Sec61 translocon complex binding [GO:0106138] (molecular function) Relationships: is a type of protein-containing complex binding [GO:0044877] Definition: Binding to a Sec61 translocon complex. References: PMID:9792704 Sources: GOC:pga